{
  "term_label": "G protein-coupled receptor signaling pathway",
  "gene_symbol": "GPR25",
  "gene_name": "Probable G-protein coupled receptor 25",
  "term_id": "GO:0007186",
  "gene": "UniProtKB:O00155"
}